{
  "gene_name": "Spermatogenesis-associated protein 25",
  "gene_symbol": "SPATA25",
  "term_id": "GO:0007283",
  "term_label": "spermatogenesis",
  "gene": "UniProtKB:Q9BR10"
}